{
  "gene": "UniProtKB:Q01449",
  "term_id": "GO:0005737",
  "gene_symbol": "MYL7",
  "gene_name": "Myosin regulatory light chain 2, atrial isoform",
  "term_label": "cytoplasm"
}